{
  "gene_symbol": "ITGB4",
  "term_id": "GO:0033627",
  "gene_name": "Integrin beta-4",
  "term_label": "cell adhesion mediated by integrin",
  "gene": "UniProtKB:P16144"
}